{
  "term_label": "extracellular space",
  "gene": "UniProtKB:P41222",
  "gene_symbol": "PTGDS",
  "term_id": "GO:0005615",
  "gene_name": "Prostaglandin-H2 D-isomerase"
}